{
  "gene_symbol": "H1-0",
  "gene": "UniProtKB:P07305",
  "term_id": "GO:0005634",
  "term_label": "nucleus",
  "gene_name": "Histone H1.0"
}